galactitol transmembrane transport [GO:0015796] (biological process) Sources: GOC:ai Relationships: is a type of GO:0015791; is a type of carbohydrate transmembrane transport [GO:0034219] Also known as: galactitol transport Definition: The directed movement of galactitol across a membrane. Galactitol is the hexitol derived by the reduction of the aldehyde group of either D- or L-galactose.